{
  "term_label": "adaptive immune response",
  "gene": "UniProtKB:P01570",
  "gene_name": "Interferon alpha-14",
  "gene_symbol": "IFNA14",
  "term_id": "GO:0002250"
}